{
  "term_label": "Unknown molecular function",
  "gene": "UniProtKB:P24311",
  "gene_name": "Cytochrome c oxidase subunit 7B, mitochondrial",
  "gene_symbol": "COX7B",
  "term_id": "UNKNOWN:0001"
}